{
  "gene_symbol": "IFNA6",
  "term_label": "B cell activation involved in immune response",
  "gene_name": "Interferon alpha-6",
  "gene": "UniProtKB:P05013",
  "term_id": "GO:0002312"
}